L-histidine conjugated cholate hydrolase activity [GO:7770008] (MF) Definition: Catalysis of the reaction: cholate + L-histidine = L-histidocholate + H2O. Relationships: is a type of amino acid conjugated cholate hydrolase activity [GO:7770003] References: PMID:38326608 Sources: RHEA:79099